{
  "gene_symbol": "CLN3",
  "gene_name": "Battenin",
  "term_id": "GO:0007040",
  "gene": "UniProtKB:Q13286",
  "term_label": "lysosome organization"
}